{
  "term_id": "GO:0071004",
  "gene_name": "Splicing factor 3A subunit 1",
  "gene": "UniProtKB:Q15459",
  "gene_symbol": "SF3A1",
  "term_label": "U2-type prespliceosome"
}